G protein-coupled neurotransmitter receptor activity involved in regulation of postsynaptic membrane potential [GO:0099579] (molecular function) Relationships: is_a G protein-coupled neurotransmitter receptor activity [GO:0099528]; is_a neurotransmitter receptor activity involved in regulation of postsynaptic membrane potential [GO:0099529]; is a type of GO:0099530 Definition: A G protein-coupled neurotransmitter receptor activity, occurring in the postsynaptic membrane, involved in regulation of postsynaptic membrane potential. Also known as: G-protein coupled neurotransmitter receptor activity involved in regulation of postsynaptic membrane potential Sources: GOC:dos